nucleoside biosynthetic process [GO:0009163] (biological process) Definition: The chemical reactions and pathways resulting in the formation of any one of a family of organic molecules consisting of a purine or pyrimidine base covalently bonded to a sugar ribose (a ribonucleoside) or deoxyribose (a deoxyribonucleoside). Sources: GOC:jl, ISBN:0140512713 Also known as: nucleoside anabolism, nucleoside biosynthesis, nucleoside formation, nucleoside synthesis Relationships: is a type of nucleoside metabolic process [GO:0009116]; is a type of nucleobase-containing small molecule biosynthetic process [GO:0034404]; is a type of glycosyl compound biosynthetic process [GO:1901659] Subtypes: purine nucleoside biosynthetic process [GO:0042451], ribonucleoside biosynthetic process [GO:0042455], nucleoside salvage [GO:0043174], deoxyribonucleoside biosynthetic process [GO:0046120], pyrimidine nucleoside biosynthetic process [GO:0046134], pyridine nucleoside biosynthetic process [GO:0071589]